{
  "gene": "UniProtKB:Q8N8D9",
  "term_label": "Unknown cellular component",
  "term_id": "UNKNOWN:0003",
  "gene_symbol": "IRF1-AS1",
  "gene_name": "Uncharacterized protein IRF1-AS1"
}